{
  "gene_symbol": "PAEP",
  "term_label": "Unknown cellular component",
  "gene": "UniProtKB:P09466",
  "gene_name": "Glycodelin",
  "term_id": "UNKNOWN:0003"
}